{
  "gene_name": "Protransforming growth factor alpha",
  "gene_symbol": "TGFA",
  "term_label": "epidermal growth factor receptor binding",
  "gene": "UniProtKB:P01135",
  "term_id": "GO:0005154"
}